septin ring organization [GO:0031106] (biological process) Relationships: is a type of septin cytoskeleton organization [GO:0032185] Definition: Control of the formation, spatial distribution, and breakdown of the septin ring. Also known as: septin ring organisation Subtypes: septin ring assembly [GO:0000921], GO:0031107, cellular bud neck septin ring organization [GO:0032186] Sources: GOC:mah